{
  "gene_name": "POTE ankyrin domain family member G",
  "term_id": "UNKNOWN:0003",
  "gene_symbol": "POTEG",
  "gene": "UniProtKB:Q6S5H5",
  "term_label": "Unknown cellular component"
}